{
  "term_id": "GO:0006511",
  "term_label": "ubiquitin-dependent protein catabolic process",
  "gene_name": "BTB_POZ domain-containing protein KCTD6",
  "gene_symbol": "KCTD6",
  "gene": "UniProtKB:Q8NC69"
}